{
  "term_id": "GO:0038117",
  "gene_symbol": "CCR7",
  "term_label": "C-C motif chemokine 19 receptor activity",
  "gene_name": "C-C chemokine receptor type 7",
  "gene": "UniProtKB:P32248"
}